{
  "term_id": "GO:0005737",
  "gene_symbol": "CAMK2B",
  "gene_name": "Calcium_calmodulin-dependent protein kinase type II subunit beta",
  "gene": "UniProtKB:Q13554",
  "term_label": "cytoplasm"
}